maintenance of alignment of postsynaptic density and presynaptic active zone [GO:0099559] (biological process) Definition: The process by which alignment between postsynaptic density and presynaptic active zone is maintained. Sources: GOC:dos Relationships: is a type of maintenance of synapse structure [GO:0099558]